{
  "term_id": "UNKNOWN:0002",
  "gene_name": "Adipocyte plasma membrane-associated protein",
  "gene_symbol": "APMAP",
  "gene": "UniProtKB:Q9HDC9",
  "term_label": "Unknown biological process"
}